{
  "gene_name": "E3 SUMO-protein ligase ZNF451",
  "term_id": "GO:0000981",
  "gene_symbol": "ZNF451",
  "gene": "UniProtKB:Q9Y4E5",
  "term_label": "DNA-binding transcription factor activity, RNA polymerase II-specific"
}